{
  "term_label": "COPI vesicle coat",
  "gene_name": "Coatomer subunit delta",
  "term_id": "GO:0030126",
  "gene": "UniProtKB:P48444",
  "gene_symbol": "ARCN1"
}